{
  "term_id": "GO:0005737",
  "term_label": "cytoplasm",
  "gene_symbol": "DNMT3A",
  "gene_name": "DNA (cytosine-5)-methyltransferase 3A",
  "gene": "UniProtKB:Q9Y6K1"
}